pyrimidine nucleoside monophosphate metabolic process [GO:0009129] (biological process) Sources: GOC:go_curators, ISBN:0198506732 Also known as: pyrimidine nucleoside monophosphate metabolism Relationships: is a type of nucleoside monophosphate metabolic process [GO:0009123] Definition: The chemical reactions and pathways involving pyrimidine nucleoside monophosphate, a compound consisting of a pyrimidine base linked to a ribose or deoxyribose sugar esterified with phosphate on the sugar. Subtypes: pyrimidine nucleoside monophosphate biosynthetic process [GO:0009130], pyrimidine nucleoside monophosphate catabolic process [GO:0009131], pyrimidine ribonucleoside monophosphate metabolic process [GO:0009173], pyrimidine deoxyribonucleoside monophosphate metabolic process [GO:0009176]